{
  "gene_name": "DNA topoisomerase 1",
  "gene": "UniProtKB:P11387",
  "term_id": "GO:0005730",
  "gene_symbol": "TOP1",
  "term_label": "nucleolus"
}